{
  "term_label": "intracellular signal transduction",
  "term_id": "GO:0035556",
  "gene_name": "MAP_microtubule affinity-regulating kinase 3",
  "gene": "UniProtKB:P27448",
  "gene_symbol": "MARK3"
}